postsynaptic spectrin-associated cytoskeleton organization [GO:0099190] (biological process) Relationships: is a type of postsynaptic cytoskeleton organization [GO:0099188] References: PMID:28576936 Sources: GOC:dos Definition: A process that is carried out at the cellular level which results in the assembly, arrangement of constituent parts, or disassembly of spectrin-associated cytoskeleton and associated proteins in the postsynapse.